RNA transmembrane transporter activity [GO:0051033] (molecular function) Subtypes: tRNA transmembrane transporter activity [GO:0051034] Relationships: is a type of GO:0051032; is part of RNA transport [GO:0050658] Sources: GOC:ai Definition: Enables the transfer of RNA, ribonucleic acid, from one side of a membrane to the other.